isotropic cell growth [GO:0051210] (biological process) Sources: GOC:ai, GOC:jid Relationships: is a type of cell growth [GO:0016049] Also known as: uniform cell growth Definition: The process in which a cell irreversibly increases in size uniformly in all directions. In general, a rounded cell morphology reflects isotropic cell growth.